{
  "gene_name": "Interleukin-1 receptor-associated kinase 4",
  "gene_symbol": "IRAK4",
  "term_label": "plasma membrane",
  "gene": "UniProtKB:Q9NWZ3",
  "term_id": "GO:0005886"
}